inactive sex chromosome [GO:0098577] (cellular component) Relationships: is a type of sex chromosome [GO:0000803] Sources: GOC:dos Definition: A sex chromosome that has been inactivated. Also known as: inactivated sex chromosome